{
  "term_label": "plasma membrane",
  "gene_symbol": "HSPA7",
  "term_id": "GO:0005886",
  "gene": "UniProtKB:P48741",
  "gene_name": "Putative heat shock 70 kDa protein 7"
}